hypothalamus gonadotrophin-releasing hormone neuron fate commitment [GO:0021887] (biological process) Relationships: is a type of cell fate commitment [GO:0045165]; is part of hypothalamus gonadotrophin-releasing hormone neuron differentiation [GO:0021886] Definition: The process in which the developmental fate of a cell becomes restricted such that it will develop into a hypothalamus neuron that releases gonadotrophin-releasing hormone. Also known as: hypothalamus gonadotropin-releasing hormone neuron fate commitment References: PMID:12626695 Sources: GOC:cls, GOC:dgh, GOC:dph, GOC:jid, GO_REF:0000021